{
  "gene": "UniProtKB:P62736",
  "term_id": "GO:0005200",
  "term_label": "structural constituent of cytoskeleton",
  "gene_name": "Actin, aortic smooth muscle",
  "gene_symbol": "ACTA2"
}